{
  "gene": "UniProtKB:Q9H0R4",
  "gene_name": "Haloacid dehalogenase-like hydrolase domain-containing protein 2",
  "term_id": "GO:0016791",
  "gene_symbol": "HDHD2",
  "term_label": "phosphatase activity"
}